{
  "term_id": "GO:0032717",
  "gene_symbol": "BPI",
  "gene_name": "Bactericidal permeability-increasing protein",
  "term_label": "negative regulation of interleukin-8 production",
  "gene": "UniProtKB:P17213"
}